{
  "gene": "UniProtKB:P09067",
  "gene_symbol": "HOXB5",
  "term_label": "nucleus",
  "term_id": "GO:0005634",
  "gene_name": "Homeobox protein Hox-B5"
}